{
  "gene": "UniProtKB:Q4U2R8",
  "gene_symbol": "SLC22A6",
  "gene_name": "Solute carrier family 22 member 6",
  "term_label": "organic anion transport",
  "term_id": "GO:0015711"
}